{
  "gene_symbol": "DEFB127",
  "term_label": "Unknown molecular function",
  "gene": "UniProtKB:Q9H1M4",
  "gene_name": "Beta-defensin 127",
  "term_id": "UNKNOWN:0001"
}